{
  "gene_symbol": "TMEM87A",
  "gene": "UniProtKB:Q8NBN3",
  "term_id": "GO:0032580",
  "term_label": "Golgi cisterna membrane",
  "gene_name": "Transmembrane protein 87A"
}